{
  "term_id": "GO:0051930",
  "gene": "UniProtKB:P15309",
  "term_label": "regulation of sensory perception of pain",
  "gene_symbol": "ACP3",
  "gene_name": "Prostatic acid phosphatase"
}